{
  "gene_symbol": "NOL6",
  "gene": "UniProtKB:Q9H6R4",
  "gene_name": "Nucleolar protein 6",
  "term_label": "rRNA processing",
  "term_id": "GO:0006364"
}